{
  "term_id": "GO:0005737",
  "term_label": "cytoplasm",
  "gene": "UniProtKB:Q96QG7",
  "gene_name": "Myotubularin-related protein 9",
  "gene_symbol": "MTMR9"
}